{
  "term_id": "UNKNOWN:0001",
  "gene_name": "NLR family member X1",
  "gene": "UniProtKB:Q86UT6",
  "term_label": "Unknown molecular function",
  "gene_symbol": "NLRX1"
}